lipoate synthase activity [GO:0016992] (molecular function) Definition: Catalysis of the reaction: protein N6-(octanoyl)lysine + 2 sulfur + 2 S-adenosyl-L-methionine = protein N6-(lipoyl)lysine + 2 L-methionine + 2 5'-deoxyadenosyl. References: PMID:18307109 Sources: EC:2.8.1.8 Also known as: lipoic acid synthase, LS, LipA, lipoyl synthase activity, protein 6-N-(octanoyl)lysine:sulfur sulfurtransferase activity, protein N6-(octanoyl)lysine:sulfur sulfurtransferase activity Relationships: is a type of GO:0016783; is part of GO:0009107